negative regulation of fibroblast growth factor receptor signaling pathway involved in ureteric bud formation [GO:2000703] (biological process) Definition: Any process that stops, prevents or reduces the frequency, rate or extent of fibroblast growth factor receptor signaling pathway involved in ureteric bud formation. Sources: GOC:mtg_kidney_jan10, GOC:obol, GOC:yaf Also known as: negative regulation of FGF receptor signaling pathway of ureteric bud formation, negative regulation of FGF receptor signalling pathway of ureteric bud formation, negative regulation of FGFR signaling pathway of ureteric bud formation, negative regulation of fibroblast growth factor receptor signaling pathway of ureteric bud formation, negative regulation of fibroblast growth factor receptor signalling pathway of ureteric bud formation Relationships: is a type of GO:0040037; is a type of GO:2000702; negatively regulates fibroblast growth factor receptor signaling pathway involved in ureteric bud formation [GO:2000699]